endocardial cushion formation [GO:0003272] (biological process) Definition: The developmental process pertaining to the initial formation of an endocardial cushion. The endocardial cushion is a specialized region of mesenchymal cells that will give rise to the heart septa and valves. References: PMID:15797462 Sources: GOC:mtg_heart Relationships: is a type of anatomical structure formation involved in morphogenesis [GO:0048646]; is part of GO:0003203